{
  "term_id": "GO:0005549",
  "gene": "UniProtKB:A6NET4",
  "gene_name": "Olfactory receptor 5K3",
  "term_label": "odorant binding",
  "gene_symbol": "OR5K3"
}